proteasome regulatory particle assembly [GO:0070682] (biological process) Relationships: is a type of proteasome assembly [GO:0043248] Also known as: proteasome regulatory complex assembly Definition: The aggregation, arrangement and bonding together of a mature, active proteasome regulatory particle complex. References: PMID:19412159 Sources: GOC:mah, GOC:rb